{
  "gene_symbol": "TBX2",
  "gene": "UniProtKB:Q13207",
  "term_id": "GO:0000981",
  "gene_name": "T-box transcription factor TBX2",
  "term_label": "DNA-binding transcription factor activity, RNA polymerase II-specific"
}